{
  "term_label": "mitochondrion",
  "gene_name": "Putative lipoyltransferase 2, mitochondrial",
  "gene_symbol": "LIPT2",
  "gene": "UniProtKB:A6NK58",
  "term_id": "GO:0005739"
}